{
  "gene": "UniProtKB:P55197",
  "gene_name": "Protein AF-10",
  "term_label": "chromatin remodeling",
  "gene_symbol": "MLLT10",
  "term_id": "GO:0006338"
}